{
  "gene_name": "Syntaxin-6",
  "term_id": "GO:0031201",
  "term_label": "SNARE complex",
  "gene": "UniProtKB:O43752",
  "gene_symbol": "STX6"
}